floral whorl formation [GO:0048458] (biological process) Definition: The process that gives rise to the floral whorl. This process pertains to the initial formation of a structure from unspecified parts. Relationships: is a type of GO:0003006; is a type of anatomical structure formation involved in morphogenesis [GO:0048646]; is part of floral whorl morphogenesis [GO:0048457] Sources: GOC:PO_curators, GOC:jid, PO:0025023